{
  "gene_name": "Putative uncharacterized protein C11orf40",
  "term_label": "Unknown molecular function",
  "gene": "UniProtKB:Q8WZ69",
  "term_id": "UNKNOWN:0001",
  "gene_symbol": "C11orf40"
}